bacteriochlorophyllide-a dehydrogenase activity [GO:0036354] (molecular function) References: PMID:8437569 Sources: RHEA:19733 Also known as: 2-desacetyl-2-hydroxyethyl bacteriochlorophyllide a dehydrogenase activity Definition: Catalysis of the reaction: 3-deacetyl-3-(1-hydroxyethyl)bacteriochlorophyllide a + NAD+ = bacteriochlorophyllide a + NADH + H+. Relationships: is a type of oxidoreductase activity, acting on the CH-OH group of donors, NAD or NADP as acceptor [GO:0016616]; is part of GO:0030494